{
  "gene_symbol": "ARID1B",
  "gene": "UniProtKB:Q8NFD5",
  "gene_name": "AT-rich interactive domain-containing protein 1B",
  "term_id": "GO:0071565",
  "term_label": "nBAF complex"
}